actin cortical patch assembly [GO:0000147] (biological process) Relationships: is a type of GO:0022607; is a type of cortical actin cytoskeleton organization [GO:0030866]; is_a actin cortical patch organization [GO:0044396] Definition: Assembly of an actin cortical patch, a discrete actin-containing structure found at the plasma membrane of fungal cells. Sources: GOC:mah Regulation: RO_0002212 by negative regulation of actin cortical patch assembly [GO:0120133]